response to acetylsalicylate [GO:1903492] (biological process) References: PMID:23392654 Sources: GOC:TermGenie, GO_REF:0000071 Definition: Any process that results in a change in state or activity of a cell or an organism (in terms of movement, secretion, enzyme production, gene expression, etc.) as a result of an aspirin (acetylsalicylate) stimulus. Aspirin is a non-steroidal anti-inflammatory drug with moA cyclooxygenase inhibitor activity. Relationships: is a type of GO:1901700